{
  "term_id": "GO:0001913",
  "term_label": "T cell mediated cytotoxicity",
  "gene_name": "Perforin-1",
  "gene": "UniProtKB:P14222",
  "gene_symbol": "PRF1"
}